{
  "gene_name": "Protein FAM91A1",
  "term_label": "vesicle tethering to Golgi",
  "gene_symbol": "FAM91A1",
  "term_id": "GO:0099041",
  "gene": "UniProtKB:Q658Y4"
}